regulation of zinc ion transmembrane transport [GO:0071580] (biological process) Definition: Any process that modulates the frequency, rate or extent of the directed movement of zinc ions (Zn2+) from one side of a membrane to the other. Sources: GOC:BHF, GOC:mah Relationships: is a type of regulation of zinc ion transport [GO:0071579]; is a type of regulation of monoatomic cation transmembrane transport [GO:1904062]; regulates zinc ion transmembrane transport [GO:0071577] Subtypes: regulation of zinc ion transmembrane import [GO:0071581], negative regulation of zinc ion transmembrane transport [GO:0071583] Also known as: regulation of zinc ion membrane transport